{
  "gene_symbol": "MRPL13",
  "term_label": "structural constituent of ribosome",
  "gene": "UniProtKB:Q9BYD1",
  "term_id": "GO:0003735",
  "gene_name": "Large ribosomal subunit protein uL13m"
}